{
  "gene_symbol": "USP17L17",
  "term_id": "GO:0005829",
  "gene_name": "Ubiquitin carboxyl-terminal hydrolase 17-like protein 17",
  "gene": "UniProtKB:D6RBQ6",
  "term_label": "cytosol"
}